{
  "gene_symbol": "CSNK1D",
  "gene": "UniProtKB:P48730",
  "term_id": "GO:0042752",
  "gene_name": "Casein kinase I isoform delta",
  "term_label": "regulation of circadian rhythm"
}